{
  "gene_name": "Protein ABHD16B",
  "term_id": "GO:0047372",
  "gene_symbol": "ABHD16B",
  "gene": "UniProtKB:Q9H3Z7",
  "term_label": "monoacylglycerol lipase activity"
}